{
  "gene_symbol": "PSMB9",
  "term_id": "GO:0043161",
  "gene": "UniProtKB:P28065",
  "gene_name": "Proteasome subunit beta type-9",
  "term_label": "proteasome-mediated ubiquitin-dependent protein catabolic process"
}